{
  "gene_name": "Putative uncharacterized protein FLJ31958",
  "term_label": "Unknown biological process",
  "term_id": "UNKNOWN:0002",
  "gene_symbol": "Q96MT0",
  "gene": "UniProtKB:Q96MT0"
}